{
  "gene": "UniProtKB:P0C0S5",
  "term_label": "nucleosome",
  "gene_name": "Histone H2A.Z",
  "gene_symbol": "H2AZ1",
  "term_id": "GO:0000786"
}